{
  "term_label": "endoplasmic reticulum membrane",
  "gene_name": "Signal recognition particle receptor subunit alpha",
  "gene": "UniProtKB:P08240",
  "term_id": "GO:0005789",
  "gene_symbol": "SRPRA"
}